{
  "gene_symbol": "TAMM41",
  "gene_name": "Phosphatidate cytidylyltransferase, mitochondrial",
  "gene": "UniProtKB:Q96BW9",
  "term_label": "mitochondrion",
  "term_id": "GO:0005739"
}